{
  "gene_name": "RNA 3'-terminal phosphate cyclase-like protein",
  "term_label": "RNA endonuclease activity",
  "term_id": "GO:0004521",
  "gene_symbol": "RCL1",
  "gene": "UniProtKB:Q9Y2P8"
}